{
  "term_id": "GO:0016607",
  "gene_name": "SNRPN upstream reading frame protein",
  "gene_symbol": "SNURF",
  "term_label": "nuclear speck",
  "gene": "UniProtKB:Q9Y675"
}